positive regulation of chronic inflammatory response [GO:0002678] (biological process) Definition: Any process that activates or increases the frequency, rate, or extent of a chronic inflammatory response. Subtypes: positive regulation of granuloma formation [GO:0002633], GO:0002876, positive regulation of chronic inflammatory response to non-antigenic stimulus [GO:0002882] Also known as: up regulation of chronic inflammatory response, up-regulation of chronic inflammatory response, upregulation of chronic inflammatory response, activation of chronic inflammatory response, stimulation of chronic inflammatory response Sources: GOC:add Relationships: is a type of regulation of chronic inflammatory response [GO:0002676]; is a type of positive regulation of inflammatory response [GO:0050729]; positively regulates chronic inflammatory response [GO:0002544]